host cell cytoplasmic vesicle membrane [GO:0044162] (cellular component) Definition: The lipid bilayer surrounding a host cell cytoplasmic vesicle. Subtypes: double membrane vesicle viral factory membrane [GO:0062242], host cell endocytic vesicle membrane [GO:0097348], host cell synaptic vesicle membrane [GO:0098585] Sources: GOC:rph Relationships: is_a host cell membrane [GO:0033644]; is a type of host cell cytoplasm part [GO:0033655]; is part of host cell cytoplasmic vesicle [GO:0044161]